{
  "gene_name": "Doublesex- and mab-3-related transcription factor 1",
  "term_label": "RNA polymerase II cis-regulatory region sequence-specific DNA binding",
  "term_id": "GO:0000978",
  "gene": "UniProtKB:Q9Y5R6",
  "gene_symbol": "DMRT1"
}